{
  "gene_symbol": "TAF4",
  "term_label": "DNA binding",
  "gene_name": "Transcription initiation factor TFIID subunit 4",
  "gene": "UniProtKB:O00268",
  "term_id": "GO:0003677"
}